{
  "gene_symbol": "TSPAN1",
  "term_id": "GO:0005886",
  "term_label": "plasma membrane",
  "gene_name": "Tetraspanin-1",
  "gene": "UniProtKB:O60635"
}